{
  "gene": "UniProtKB:O00443",
  "term_label": "cytoplasm",
  "gene_symbol": "PIK3C2A",
  "gene_name": "Phosphatidylinositol 4-phosphate 3-kinase C2 domain-containing subunit alpha",
  "term_id": "GO:0005737"
}